{
  "gene_symbol": "FERMT1",
  "term_label": "integrin binding",
  "gene": "UniProtKB:Q9BQL6",
  "gene_name": "Fermitin family homolog 1",
  "term_id": "GO:0005178"
}